{
  "gene": "UniProtKB:Q92963",
  "gene_symbol": "RIT1",
  "term_id": "GO:0005886",
  "term_label": "plasma membrane",
  "gene_name": "GTP-binding protein Rit1"
}